{
  "gene": "UniProtKB:Q6IQ20",
  "term_id": "GO:0005737",
  "gene_symbol": "NAPEPLD",
  "term_label": "cytoplasm",
  "gene_name": "N-acyl-phosphatidylethanolamine-hydrolyzing phospholipase D"
}